{
  "gene_symbol": "CD38",
  "term_label": "plasma membrane",
  "gene": "UniProtKB:P28907",
  "term_id": "GO:0005886",
  "gene_name": "ADP-ribosyl cyclase_cyclic ADP-ribose hydrolase 1"
}